olfactory pit development [GO:0060166] (BP) Relationships: is a type of anatomical structure development [GO:0048856]; is part of nose development [GO:0043584] Definition: The biological process whose specific outcome is the progression of the olfactory pit from an initial condition to its mature state. This process begins with the formation of the olfactory pit, which is an indentation of the olfactory placode, and ends when the pits hollows out to form the nasopharynx. Sources: GOC:dph, ISBN:0124020607